D-mannitol oxidase activity [GO:0050581] (molecular function) Relationships: is a type of GO:0016899 Also known as: D-arabinitol oxidase activity, D-arabitol oxidase activity, mannitol oxidase activity, mannitol:oxygen oxidoreductase (cyclizing) Sources: EC:1.1.3.40, MetaCyc:1.1.3.40-RXN Definition: Catalysis of the reaction: mannitol + O2 = mannose + H2O2.